{
  "term_label": "Unknown biological process",
  "gene_symbol": "MIS18BP1",
  "gene_name": "Mis18-binding protein 1",
  "gene": "UniProtKB:Q6P0N0",
  "term_id": "UNKNOWN:0002"
}